{
  "gene_name": "Putative histone H2B type 2-C",
  "gene_symbol": "H2BC20P",
  "term_id": "GO:0000786",
  "gene": "UniProtKB:Q6DN03",
  "term_label": "nucleosome"
}